{
  "gene": "UniProtKB:Q86X60",
  "gene_symbol": "FAM72B",
  "term_id": "GO:0005829",
  "gene_name": "Protein FAM72B",
  "term_label": "cytosol"
}